double membrane vesicle viral factory [GO:0039718] (cellular component) Also known as: DMV viral factory References: PMID:22440839 Sources: VZ:1951 Definition: A cytoplasmic viral factory that consists of a double-membrane bound vesicle. Has a diameter of 200-300nm and is derived from the endoplasmic reticulum or Golgi apparatus. Produced by Picornaviridae, Nidovirales, Arteriviridae and Coronaviridae. Relationships: is a type of cytoplasmic viral factory [GO:0039714]